{
  "gene_name": "Histone-binding protein RBBP7",
  "term_id": "GO:0006355",
  "term_label": "regulation of DNA-templated transcription",
  "gene_symbol": "RBBP7",
  "gene": "UniProtKB:Q16576"
}